complex laminated body [GO:1990012] (CC) Definition: A cytoplasmic inclusion body found in some lateral geniculate neurons and composed of sheets of tubules (25 nm in diameter) separated by dense material (about 75 nm wide), which together with the tubules whorl give a structure resembling a fingerprint. Sources: NIF_Subcellular:nlx_151681 Relationships: is a type of GO:1990011 Also known as: CLB